ciliary microtubule quartet [GO:0120260] (cellular component) References: PMID:19299460, PMID:32518185 Sources: DOI:10.5772/66859, GOC:ach, GOC:krc Also known as: ciliary MtQ Note: Note that cilia and eukaryotic flagella are deemed to be equivalent. In diplomonad species, such as Giardia, the axoneme may extend intracellularly up to 5um away from the plane of the plasma membrane. Definition: A set of four specialized microtubules that originates from the basal bodies and wraps around the ciliary pocket membrane, likely supporting its distinct flask shape. Relationships: is a type of cellular anatomical structure [GO:0110165]; is part of cytoskeleton [GO:0005856]; is part of GO:0005929; has part GO:0005874